UDP-N-acetylglucosamine transferase complex [GO:0043541] (cellular component) Definition: A multienzyme, heterooligomeric complex involved in dolichyl-linked oligosaccharide synthesis. In yeast the complex is composed of Alg7p, which catalyzes the first step (GlcNAc1-PP-Dol from dolichol-phosphate and UDP-GlcNAc), and Alg13p plus Alg14p, the catalytic and anchoring subunits respectively, which together catalyze the second step (GlcNAc2-PP-dolichol from GlcNAc1-PP-Dol and UDP-GlcNAc) of dolichyl-linked oligosaccharide synthesis. References: PMID:19129246 Sources: GOC:rn Relationships: is a type of GO:0061695; is_a membrane protein complex [GO:0098796]; is a type of endoplasmic reticulum protein-containing complex [GO:0140534]; BFO_0000050 GO:0005789